{
  "term_id": "UNKNOWN:0002",
  "term_label": "Unknown biological process",
  "gene_symbol": "C16orf89",
  "gene": "UniProtKB:Q6UX73",
  "gene_name": "UPF0764 protein C16orf89"
}